{
  "term_label": "Unknown molecular function",
  "gene_symbol": "LY6G5C",
  "term_id": "UNKNOWN:0001",
  "gene": "UniProtKB:Q5SRR4",
  "gene_name": "Lymphocyte antigen 6 complex locus protein G5c"
}